negative regulation of nuclear-transcribed mRNA catabolic process, nonsense-mediated decay [GO:2000623] (biological process) Relationships: is a type of negative regulation of mRNA catabolic process [GO:1902373]; is a type of GO:2000622; negatively regulates nuclear-transcribed mRNA catabolic process, nonsense-mediated decay [GO:0000184] Also known as: negative regulation of mRNA breakdown, nonsense-mediated decay, negative regulation of mRNA catabolic process, nonsense-mediated, negative regulation of mRNA catabolism, nonsense-mediated, negative regulation of mRNA degradation, nonsense-mediated decay, negative regulation of nonsense-mediated mRNA decay, negative regulation of nuclear mRNA catabolic process, nonsense-mediated decay Sources: GOC:obol Definition: Any process that stops, prevents or reduces the frequency, rate or extent of nuclear-transcribed mRNA catabolic process, nonsense-mediated decay.